isoflavone 3'-hydroxylase activity [GO:0048000] (molecular function) Definition: Catalysis of the reaction: formononetin + NADPH + O2 = calycosin + NADP+ + H2O. Sources: EC:1.14.14.88 Also known as: formononetin,NADPH:oxygen oxidoreductase (3'-hydroxylating), isoflavone 3'-monooxygenase activity Relationships: is a type of GO:0016709